pantothenate metabolic process [GO:0015939] (biological process) Definition: The chemical reactions and pathways involving pantothenate, the anion of pantothenic acid, the amide of beta-alanine and pantoic acid. It is a B complex vitamin that is a constituent of coenzyme A and is distributed ubiquitously in foods. Also known as: pantothenate metabolism, vitamin B5 metabolic process, vitamin B5 metabolism Relationships: is_a modified amino acid metabolic process [GO:0006575]; is a type of GO:0032787; is_a amide metabolic process [GO:0043603] Subtypes: pantothenate biosynthetic process [GO:0015940], pantothenate catabolic process [GO:0015941], acetyl-CoA biosynthetic process from pantothenate [GO:1990181] Sources: GOC:ai, ISBN:0721662544